{
  "gene": "UniProtKB:C9JE40",
  "term_id": "GO:0000290",
  "gene_name": "Protein PAT1 homolog 2",
  "term_label": "deadenylation-dependent decapping of nuclear-transcribed mRNA",
  "gene_symbol": "PATL2"
}